{
  "gene": "UniProtKB:P37231",
  "gene_name": "Peroxisome proliferator-activated receptor gamma",
  "term_label": "intracellular receptor signaling pathway",
  "term_id": "GO:0030522",
  "gene_symbol": "PPARG"
}